sphingolipid C4-monooxygenase activity [GO:0102772] (molecular function) Definition: Catalysis of the reaction: a dihydroceramide + 2 Fe(II)-[cytochrome b5] + 2 H+ + O2 = a phytoceramide + 2 Fe(III)-[cytochrome b5] + H2O. Relationships: is a type of oxidoreductase activity, acting on paired donors, with incorporation or reduction of molecular oxygen, another compound as one donor, and incorporation of one atom of oxygen [GO:0016716] Sources: EC:1.14.18.5, GOC:pz Also known as: sphingolipid long-chain base 4-hydroxylase activity